regulation of D-aspartate import across plasma membrane [GO:0140215] (biological process) Subtypes: negative regulation of D-aspartate import across plasma membrane [GO:0140216], positive regulation of D-aspartate import across plasma membrane [GO:0140217] References: PMID:27663541 Definition: Any process that modulates the frequency, rate or extent of the directed import of D-aspartate from the extracellular region across the plasma membrane and into the cytosol. Relationships: is a type of GO:0010958; is a type of regulation of organic acid transport [GO:0032890]; regulates D-aspartate import across plasma membrane [GO:0070779]